{
  "term_label": "Unknown biological process",
  "gene_symbol": "TMEM52",
  "gene": "UniProtKB:Q8NDY8",
  "gene_name": "Transmembrane protein 52",
  "term_id": "UNKNOWN:0002"
}